muscle thin filament tropomyosin [GO:0005862] (cellular component) Sources: ISBN:0815316194 Definition: A form of the tropomyosin dimer found associated with actin and the troponin complex in muscle thin filaments. Relationships: is a type of protein-containing complex [GO:0032991]; is part of striated muscle thin filament [GO:0005865]